calcium ion transport into cytosol [GO:0060402] (biological process) Relationships: is a type of positive regulation of cytosolic calcium ion concentration [GO:0007204]; is a type of calcium ion transmembrane import into cytosol [GO:0097553] Regulation: regulated by regulation of calcium ion transport into cytosol [GO:0010522]; negatively regulated by negative regulation of calcium ion transport into cytosol [GO:0010523]; positively regulated by GO:0010524 Definition: The directed movement of calcium ions (Ca2+) into the cytosol. Sources: GOC:dph, GOC:tb